{
  "gene_name": "Olfactory receptor 52A4",
  "term_label": "olfactory receptor activity",
  "gene_symbol": "OR52A4P",
  "gene": "UniProtKB:A6NMU1",
  "term_id": "GO:0004984"
}